{
  "gene_symbol": "MCEE",
  "gene_name": "Methylmalonyl-CoA epimerase, mitochondrial",
  "term_id": "UNKNOWN:0003",
  "term_label": "Unknown cellular component",
  "gene": "UniProtKB:Q96PE7"
}